{
  "term_label": "negative chemotaxis",
  "gene_name": "Slit homolog 1 protein",
  "term_id": "GO:0050919",
  "gene": "UniProtKB:O75093",
  "gene_symbol": "SLIT1"
}